regulation of protein localization to chromatin [GO:1905634] (biological process) Definition: Any process that modulates the frequency, rate or extent of protein localization to chromatin. Also known as: regulation of protein localisation to chromatin References: PMID:20889714 Sources: GOC:TermGenie, GO_REF:0000058 Relationships: is a type of regulation of protein localization [GO:0032880]; regulates GO:0071168 Subtypes: negative regulation of protein localization to chromatin [GO:0120186], positive regulation of protein localization to chromatin [GO:0120187]